UDP-N-acetylglucosamine-undecaprenyl-phosphate N-acetylglucosaminephosphotransferase activity [GO:0036380] (molecular function) Sources: EC:2.7.8.33, GOC:rs Definition: Catalysis of the reaction: UDP-N-acetyl-alpha-D-glucosamine + ditrans,octacis-undecaprenyl phosphate = UMP + N-acetyl-alpha-D-glucosaminyldiphospho-ditrans,octacis-undecaprenol. Also known as: GlcNAc-P-P-Und synthase activity, UDP-GIcNAc:undecaprenyl phosphate N-acetylglucosaminyl 1-P transferase activity, UDP-GlcNAc:undecaprenyl-phosphate GlcNAc-1-phosphate transferase activity, UDP-N-acetyl-D-glucosamine:ditrans,octacis-undecaprenyl phosphate N-acetyl-D-glucosaminephosphotransferase activity, UDP-N-acetylglucosamine:undecaprenyl-phosphate GlcNAc-1-phosphate transferase activity Relationships: is a type of phosphotransferase activity, for other substituted phosphate groups [GO:0016780]